{
  "gene_symbol": "DOP1A",
  "term_id": "GO:0005802",
  "term_label": "trans-Golgi network",
  "gene_name": "Protein dopey-1",
  "gene": "UniProtKB:Q5JWR5"
}